regulation of L-lysine import across plasma membrane [GO:1905008] (biological process) Subtypes: negative regulation of L-lysine import across plasma membrane [GO:1905009], GO:1905010 References: PMID:7499219 Sources: GOC:TermGenie, GO_REF:0000058 Also known as: regulation of lysine import, regulation of L-lysine import into cell, regulation of lysine uptake Relationships: is a type of regulation of amino acid import across plasma membrane [GO:0010958]; is a type of regulation of organic acid transport [GO:0032890]; regulates L-lysine import across plasma membrane [GO:0097639] Definition: Any process that modulates the frequency, rate or extent of L-lysine import into cell.